{
  "term_id": "GO:0005737",
  "gene": "UniProtKB:Q969Q4",
  "term_label": "cytoplasm",
  "gene_name": "ADP-ribosylation factor-like protein 11",
  "gene_symbol": "ARL11"
}